phosphatidylethanolamine metabolic process [GO:0046337] (biological process) Definition: The chemical reactions and pathways involving phosphatidylethanolamine, any of a class of glycerophospholipids in which a phosphatidyl group is esterified to the hydroxyl group of ethanolamine. It is a major structural phospholipid in mammalian systems. It tends to be more abundant than phosphatidylcholine in the internal membranes of the cell and is an abundant component of prokaryotic membranes. Relationships: is a type of glycerophospholipid metabolic process [GO:0006650] Also known as: phosphatidylethanolamine metabolism Subtypes: phosphatidylethanolamine biosynthetic process [GO:0006646], GO:0046338, GO:0070292 Sources: GOC:curators, ISBN:0198506732 Regulation: regulated by regulation of phosphatidylethanolamine metabolic process [GO:0150175]